diol catabolic process [GO:0034313] (biological process) Relationships: is a type of diol metabolic process [GO:0034311]; is a type of GO:0046174 Definition: The chemical reactions and pathways resulting in the breakdown of a diol, any alcohol containing two hydroxyl groups attached to saturated carbon atoms. Sources: GOC:mah Subtypes: glycol catabolic process [GO:0042846], GO:0046147, sphingosine catabolic process [GO:0051872], asperfuranone catabolic process [GO:1900553], (+)-secoisolariciresinol catabolic process [GO:1902134], (-)-secoisolariciresinol catabolic process [GO:1902137] Also known as: dihydric alcohol catabolic process, diol breakdown, diol catabolism, diol degradation